flavonol metabolic process [GO:0051554] (biological process) Also known as: flavonol metabolism References: PMID:11402179 Definition: The chemical reactions and pathways involving flavonols, a member of a class of vascular pigments formed by consecutive oxidative processes from the flavonoid intermediates flavanones and dihydroflavonols. Flavonols are the most widespread of the flavonoids and have a wide array of physiological activities. Relationships: is a type of GO:0051552 Subtypes: flavonol biosynthetic process [GO:0051555]